{
  "gene": "UniProtKB:Q9UBI6",
  "gene_name": "Guanine nucleotide-binding protein G(I)_G(S)_G(O) subunit gamma-12",
  "term_id": "GO:0005834",
  "gene_symbol": "GNG12",
  "term_label": "heterotrimeric G-protein complex"
}